{
  "gene_symbol": "TUBGCP4",
  "term_label": "microtubule minus-end binding",
  "gene": "UniProtKB:Q9UGJ1",
  "gene_name": "Gamma-tubulin complex component 4",
  "term_id": "GO:0051011"
}